{
  "term_label": "DNA-binding transcription factor activity, RNA polymerase II-specific",
  "gene": "UniProtKB:Q9NP62",
  "gene_name": "Chorion-specific transcription factor GCMa",
  "term_id": "GO:0000981",
  "gene_symbol": "GCM1"
}